regulation of sensory perception of sweet taste [GO:1904656] (biological process) Definition: Any process that modulates the frequency, rate or extent of sensory perception of sweet taste. References: PMID:1716172 Sources: GOC:TermGenie, GOC:mr, GO_REF:0000058 Subtypes: negative regulation of sensory perception of sweet taste [GO:1904657], positive regulation of sensory perception of sweet taste [GO:1904658] Also known as: regulation of sweet taste perception Relationships: is a type of regulation of sensory perception [GO:0051931]; regulates sensory perception of sweet taste [GO:0050916]